{
  "gene_name": "Caspase recruitment domain-containing protein 18",
  "term_label": "Unknown biological process",
  "gene": "UniProtKB:P57730",
  "gene_symbol": "CARD18",
  "term_id": "UNKNOWN:0002"
}